formyl-methanofuran dehydrogenase (molybdenum enzyme) complex [GO:0044676] (CC) References: PMID:1915887, PMID:8954165 Sources: GOC:mengo_curators Relationships: is a type of GO:1902494 Definition: A protein complex consisting of three polypeptides which also contains molybdenum, a molybdopterin guanine dinucleotide and iron-sulfur clusters. This protein complex catalyzes the reversible conversion of CO2 and methanofuran to formylmethanofuran during methanogenesis.